{
  "gene_name": "Beta-enolase",
  "gene_symbol": "ENO3",
  "term_label": "phosphopyruvate hydratase complex",
  "gene": "UniProtKB:P13929",
  "term_id": "GO:0000015"
}